sphingoid catabolic process [GO:0046521] (biological process) Sources: ISBN:0198506732 Subtypes: sphingosine catabolic process [GO:0051872] Relationships: is a type of sphingolipid catabolic process [GO:0030149]; is_a sphingoid metabolic process [GO:0046519] Also known as: sphingoid breakdown, sphingoid catabolism, sphingoid degradation Definition: The chemical reactions and pathways resulting in the breakdown of sphingoids, any of a class of compounds comprising sphinganine and its homologues and stereoisomers, and derivatives of these compounds.